{
  "gene": "UniProtKB:Q400G9",
  "gene_symbol": "AMZ1",
  "term_id": "UNKNOWN:0002",
  "gene_name": "Archaemetzincin-1",
  "term_label": "Unknown biological process"
}